{
  "term_label": "nucleic acid binding",
  "term_id": "GO:0003676",
  "gene_symbol": "YBX2",
  "gene_name": "Y-box-binding protein 2",
  "gene": "UniProtKB:Q9Y2T7"
}